{
  "gene": "UniProtKB:Q14249",
  "term_id": "GO:0005634",
  "gene_symbol": "ENDOG",
  "gene_name": "Endonuclease G, mitochondrial",
  "term_label": "nucleus"
}